{
  "gene": "UniProtKB:Q9H1U9",
  "gene_name": "Mitochondrial nicotinamide adenine dinucleotide transporter SLC25A51",
  "term_id": "GO:0051724",
  "gene_symbol": "SLC25A51",
  "term_label": "NAD transmembrane transporter activity"
}